{
  "gene_name": "Probable G-protein coupled receptor 148",
  "gene": "UniProtKB:Q8TDV2",
  "term_id": "GO:0004984",
  "gene_symbol": "GPR148",
  "term_label": "olfactory receptor activity"
}